{
  "term_label": "Unknown molecular function",
  "gene_name": "Uncharacterized protein C1orf21",
  "term_id": "UNKNOWN:0001",
  "gene": "UniProtKB:Q9H246",
  "gene_symbol": "C1orf21"
}